{
  "gene": "UniProtKB:Q9UHE5",
  "gene_symbol": "NAT8",
  "gene_name": "N-acetyltransferase 8",
  "term_label": "N-acetyltransferase activity",
  "term_id": "GO:0008080"
}